{
  "gene_symbol": "B3GAT3",
  "gene": "UniProtKB:O94766",
  "term_id": "GO:0050650",
  "gene_name": "Galactosylgalactosylxylosylprotein 3-beta-glucuronosyltransferase 3",
  "term_label": "chondroitin sulfate proteoglycan biosynthetic process"
}